L-threonylcarbamoyladenylate synthase [GO:0061710] (molecular function) Sources: EC:2.7.7.87 Relationships: is a type of GO:0016779 Definition: Catalysis of the reaction: L-threonine + ATP + bicarbonate = L-threonylcarbamoyladenylate + diphosphate + H2O.